{
  "gene": "UniProtKB:Q96HY6",
  "term_label": "cartilage development",
  "term_id": "GO:0051216",
  "gene_symbol": "DDRGK1",
  "gene_name": "DDRGK domain-containing protein 1"
}